{
  "term_id": "UNKNOWN:0002",
  "gene_name": "Coiled-coil domain-containing protein 85C",
  "gene_symbol": "CCDC85C",
  "term_label": "Unknown biological process",
  "gene": "UniProtKB:A6NKD9"
}